1,1,1-trichloro-2,2-bis-(4-chlorophenyl)ethane catabolic process [GO:0042188] (biological process) Sources: GOC:jl Definition: The chemical reactions and pathways resulting in the breakdown of 1,1,1-trichloro-2,2-bis-(4-chlorophenyl)ethane (DDT), a chlorinated broad spectrum contact insecticide. Also known as: 1,1,1-trichloro-2,2-bis-(4-chlorophenyl)ethane breakdown, 1,1,1-trichloro-2,2-bis-(4-chlorophenyl)ethane catabolism, 1,1,1-trichloro-2,2-bis-(4-chlorophenyl)ethane degradation, DDT catabolic process, DDT catabolism Relationships: is a type of 1,1,1-trichloro-2,2-bis-(4-chlorophenyl)ethane metabolic process [GO:0018977]; is a type of GO:0042205; is a type of insecticide catabolic process [GO:0046701]